{
  "term_id": "GO:0043195",
  "gene_symbol": "SLC18A3",
  "term_label": "terminal bouton",
  "gene": "UniProtKB:Q16572",
  "gene_name": "Vesicular acetylcholine transporter"
}